{
  "gene_symbol": "ATP4A",
  "term_id": "GO:0006883",
  "term_label": "intracellular sodium ion homeostasis",
  "gene_name": "Potassium-transporting ATPase alpha chain 1",
  "gene": "UniProtKB:P20648"
}